{
  "gene_name": "Activin receptor type-2A",
  "term_label": "pattern specification process",
  "gene": "UniProtKB:P27037",
  "term_id": "GO:0007389",
  "gene_symbol": "ACVR2A"
}